{
  "gene_symbol": "KCNE1",
  "gene_name": "Potassium voltage-gated channel subfamily E member 1",
  "term_label": "potassium ion export across plasma membrane",
  "gene": "UniProtKB:P15382",
  "term_id": "GO:0097623"
}